arachidonate-CoA ligase activity [GO:0047676] (MF) Relationships: is a type of GO:0004467 Definition: Catalysis of the reaction: arachidonate + ATP + CoA = AMP + arachidonoyl-CoA + diphosphate + H+. Sources: RHEA:19713 Also known as: arachidonate:CoA ligase (AMP-forming), arachidonoyl-CoA synthetase activity